{
  "term_id": "UNKNOWN:0003",
  "gene": "UniProtKB:Q6ZSV7",
  "gene_name": "Putative uncharacterized protein FLJ45177",
  "gene_symbol": "Q6ZSV7",
  "term_label": "Unknown cellular component"
}